cytoplasmic alanyl-tRNA aminoacylation [GO:1990762] (biological process) Relationships: is a type of alanyl-tRNA aminoacylation [GO:0006419]; is part of cytoplasmic translation [GO:0002181] Sources: GOC:vw Definition: The process of coupling alanine to alanyl-tRNA, catalyzed by alanyl-tRNA synthetase involved in cytoplasmic translation.